positive regulation of DNA endoreduplication [GO:0032877] (biological process) Definition: Any process that activates or increases the frequency, rate or extent of DNA endoreduplication. Sources: GOC:mah Also known as: positive regulation of DNA endoreplication, positive regulation of DNA re-duplication, up regulation of DNA endoreduplication, up-regulation of DNA endoreduplication, upregulation of DNA endoreduplication, activation of DNA endoreduplication, stimulation of DNA endoreduplication Relationships: is a type of regulation of DNA endoreduplication [GO:0032875]; is a type of positive regulation of cell cycle process [GO:0090068]; is a type of positive regulation of DNA-templated DNA replication [GO:2000105]; positively regulates DNA endoreduplication [GO:0042023]